{
  "gene": "UniProtKB:O75381",
  "term_id": "GO:0016560",
  "term_label": "protein import into peroxisome matrix, docking",
  "gene_name": "Peroxisomal membrane protein PEX14",
  "gene_symbol": "PEX14"
}